(2R)-2-hydroxyacid dehydrogenase (NADP+) activity [GO:0050578] (molecular function) Also known as: (R)-2-hydroxyacid:NAD(P)+ oxidoreductase activity, (R)-sulfolactate:NAD(P)(+) oxidoreductase activity, (R)-sulfolactate:NAD(P)+ oxidoreductase activity, L-sulfolactate dehydrogenase activity Relationships: is a type of oxidoreductase activity, acting on the CH-OH group of donors, NAD or NADP as acceptor [GO:0016616]; is a type of (2R)-oxo-acid reductase activity [GO:0033719] Definition: Catalysis of the reaction: a (2R)-2-hydroxycarboxylate + NADP+ = a 2-oxocarboxylate + NADPH + H+. Sources: RHEA:35735